{
  "gene_symbol": "USP26",
  "term_label": "cytosol",
  "gene_name": "Ubiquitin carboxyl-terminal hydrolase 26",
  "term_id": "GO:0005829",
  "gene": "UniProtKB:Q9BXU7"
}